{
  "gene": "UniProtKB:O94966",
  "term_label": "regulation of protein stability",
  "gene_name": "Ubiquitin carboxyl-terminal hydrolase 19",
  "term_id": "GO:0031647",
  "gene_symbol": "USP19"
}